regulation of mature B cell apoptotic process [GO:0002905] (biological process) Subtypes: GO:0002906, GO:0002907 Also known as: regulation of mature B cell apoptosis Sources: GOC:add, GOC:mtg_apoptosis Relationships: is a type of regulation of immune system process [GO:0002682]; is a type of regulation of B cell apoptotic process [GO:0002902]; regulates GO:0002901 Definition: Any process that modulates the frequency, rate, or extent of mature B cell apoptotic process.